pyrimidine-containing compound biosynthetic process [GO:0072528] (biological process) Sources: GOC:mah Definition: The chemical reactions and pathways resulting in the formation of a pyrimidine-containing compound, i.e. any compound that contains pyrimidine or a formal derivative thereof. Subtypes: GO:0006221, pyrimidine-containing compound salvage [GO:0008655], pyrimidine nucleobase biosynthetic process [GO:0019856], thiamine-containing compound biosynthetic process [GO:0042724], pyrimidine nucleoside biosynthetic process [GO:0046134] Relationships: is a type of biosynthetic process [GO:0009058]; is a type of pyrimidine-containing compound metabolic process [GO:0072527] Also known as: pyrimidine and derivative biosynthetic process, pyrimidine-containing compound anabolism, pyrimidine-containing compound biosynthesis, pyrimidine-containing compound formation, pyrimidine-containing compound synthesis